{
  "gene_symbol": "HLA-E",
  "term_id": "GO:0030881",
  "term_label": "beta-2-microglobulin binding",
  "gene_name": "HLA class I histocompatibility antigen, alpha chain E",
  "gene": "UniProtKB:P13747"
}